apocarotenoid biosynthetic process [GO:0043289] (biological process) Definition: The chemical reactions and pathways resulting in the formation of apocarotenoids by the oxidative cleavage of carotenoids. Many apocarotenoids are biologically important e.g. retinal and abscisic acid. References: PMID:27485225 Sources: GOC:jl Also known as: apo carotenoid biosynthetic process, apocarotenoid anabolism, apocarotenoid biosynthesis, apocarotenoid formation, apocarotenoid synthesis Relationships: is a type of isoprenoid biosynthetic process [GO:0008299] Subtypes: abscisic acid biosynthetic process [GO:0009688], GO:0010379